UDP-N-acetylglucosamine-lysosomal-enzyme N-acetylglucosaminephosphotransferase complex [GO:0070622] (cellular component) Definition: A protein complex that possesses UDP-N-acetylglucosamine-lysosomal-enzyme N-acetylglucosaminephosphotransferase activity; the bovine complex contains disulfide-linked homodimers of 166- and 51-kDa subunits and two identical, noncovalently associated 56-kDa subunits. References: PMID:8940155 Sources: GOC:mah Also known as: UDP-N-acetylglucosamine:lysosomal-enzyme N-acetylglucosamine-1-phosphotransferase complex, N-acetylglucosamine-1-phosphotransferase complex Relationships: is a type of transferase complex, transferring phosphorus-containing groups [GO:0061695]; is part of lysosome [GO:0005764]